{
  "gene_symbol": "GPX3",
  "gene": "UniProtKB:P22352",
  "gene_name": "Glutathione peroxidase 3",
  "term_id": "GO:0042744",
  "term_label": "hydrogen peroxide catabolic process"
}